{
  "term_id": "GO:0007420",
  "gene_symbol": "PBX2",
  "gene_name": "Pre-B-cell leukemia transcription factor 2",
  "gene": "UniProtKB:P40425",
  "term_label": "brain development"
}